photoreceptor distal connecting cilium [GO:0120206] (cellular component) Also known as: DCC, photoreceptor DCC Definition: The distal region of the photoreceptor connecting cilium is structurally unique to the photoreceptor and is maintained by retina-specific protein, SPATA7, and its interacting partners RPGR and RPGRIP1. It is essential for photoreceptor sensory cilium stability. References: PMID:29899041 Sources: GOC:krc Relationships: is a type of cellular anatomical structure [GO:0110165]; BFO_0000050 photoreceptor connecting cilium [GO:0032391]